sinapine esterase activity [GO:0050285] (molecular function) Definition: Catalysis of the reaction: O-sinapoylcholine + H2O = choline + H+ + sinapate. Sources: EC:3.1.1.49, RHEA:10016 Also known as: aromatic choline esterase activity, sinapoylcholine sinapohydrolase activity Relationships: is a type of carboxylic ester hydrolase activity [GO:0052689]